phenylacetate 2-hydroxylase activity [GO:0018631] (MF) Definition: Catalysis of the reaction: 2-phenylacetate + O2 + reduced [NADPH--hemoprotein reductase] = (2-hydroxyphenyl)acetate + H+ + H2O + oxidized [NADPH--hemoprotein reductase]. Sources: RHEA:53392 Relationships: is a type of oxidoreductase activity, acting on paired donors, with incorporation or reduction of molecular oxygen, reduced flavin or flavoprotein as one donor, and incorporation of one atom of oxygen [GO:0016712] Also known as: phenylacetate hydroxylase activity